1,2-propanediol catabolic process [GO:0051144] (biological process) Regulation: positively regulated by positive regulation of 1,2-propanediol catabolic process [GO:0160161] References: PMID:12700259 Relationships: is a type of GO:0042846 Definition: The chemical reactions and pathways resulting in the breakdown of propanediol, a sweet, colorless, viscous, hygroscopic liquid with the formula CH3-CHOH-CH2OH. Also known as: propanediol catabolic process, 1,2-dihydroxypropane catabolic process, 1,2-dihydroxypropane catabolism, propanediol breakdown, propanediol catabolism, propanediol degradation, propylene glycol catabolic process, propylene glycol catabolism